{
  "gene_symbol": "SLC27A5",
  "term_id": "GO:0004467",
  "gene_name": "Long-chain fatty acid transport protein 5",
  "gene": "UniProtKB:Q9Y2P5",
  "term_label": "long-chain fatty acid-CoA ligase activity"
}